negative regulation of embryonic development [GO:0045992] (biological process) Subtypes: GO:0061185, negative regulation of gastrulation [GO:2000542] Definition: Any process that stops, prevents, or reduces the frequency, rate or extent of embryonic development. Relationships: is a type of regulation of embryonic development [GO:0045995]; is a type of GO:0051093; is a type of negative regulation of multicellular organismal process [GO:0051241]; negatively regulates embryo development [GO:0009790] Also known as: down regulation of embryonic development, down-regulation of embryonic development, downregulation of embryonic development, inhibition of embryonic development Sources: GOC:go_curators